{
  "gene_name": "Zinc finger protein 268",
  "term_label": "negative regulation of transcription by RNA polymerase II",
  "term_id": "GO:0000122",
  "gene_symbol": "ZNF268",
  "gene": "UniProtKB:Q14587"
}